pole plasm mitochondrial lrRNA localization [GO:0019096] (biological process) Relationships: is_a pole plasm mitochondrial rRNA localization [GO:0019095] Sources: ISBN:0879694238 Definition: Any process in which mitochondrial large ribosomal RNA is transported to, or maintained in, the oocyte pole plasm. An example of this is found in Drosophila melanogaster. Also known as: establishment and maintenance of mitochondrial lrRNA localization in pole plasm, oocyte pole plasm mitochondrial lrRNA localization, pole plasm mitochondrial lrRNA localisation